laminin receptor activity [GO:0005055] (molecular function) Definition: Combining with a laminin, a glycoprotein that constitutes the majority of proteins in the basement membrane, to initiate a change in cell activity. Note: Note that this term represents an activity and not a gene product. Consider also annotating to the molecular function terms 'cell adhesion molecule binding ; GO:0050839' and 'receptor binding ; GO:0005102' and the biological process term 'cell adhesion ; GO:0007155'. References: PMID:2970671 Sources: GOC:ai Relationships: is a type of cell adhesion mediator activity [GO:0098631]; BFO_0000051 laminin binding [GO:0043236]